Fused-Smurf ubiquitin ligase complex [GO:1990353] (cellular component) Relationships: is a type of ubiquitin ligase complex [GO:0000151] Note: An example of this is FUSED in Drosophila melanogaster (UniProt symbol P23647) in PMID:21145463 (inferred from direct assay). References: PMID:21145463 Sources: GOC:bhm Definition: A ubiquitin ligase complex. In D. melanogaster, it regulates ubiquitination and proteolysis of the BMP receptor Thickveins in cystoblasts, potentially by controlling Tkv ubiquitination and degradation.